{
  "term_label": "Unknown biological process",
  "gene_symbol": "TST",
  "gene": "UniProtKB:Q16762",
  "term_id": "UNKNOWN:0002",
  "gene_name": "Thiosulfate sulfurtransferase"
}